{
  "gene_name": "Integral membrane protein GPR137",
  "gene": "UniProtKB:Q96N19",
  "gene_symbol": "GPR137",
  "term_id": "GO:0010506",
  "term_label": "regulation of autophagy"
}